{
  "term_label": "Unknown cellular component",
  "gene": "UniProtKB:Q9UHR6",
  "gene_symbol": "ZNHIT2",
  "term_id": "UNKNOWN:0003",
  "gene_name": "Zinc finger HIT domain-containing protein 2"
}